{
  "term_label": "Unknown molecular function",
  "gene": "UniProtKB:Q9HBX3",
  "gene_symbol": "SND1-IT1",
  "term_id": "UNKNOWN:0001",
  "gene_name": "Uncharacterized protein encoded by SND1-IT1"
}